{
  "gene": "UniProtKB:A0A075B6I1",
  "gene_symbol": "IGLV4-60",
  "gene_name": "Immunoglobulin lambda variable 4-60",
  "term_id": "GO:0019814",
  "term_label": "immunoglobulin complex"
}